negative regulation of phosphatidylcholine biosynthetic process [GO:2001246] (biological process) Sources: GOC:obol Definition: Any process that stops, prevents or reduces the frequency, rate or extent of phosphatidylcholine biosynthetic process. Relationships: is a type of negative regulation of phospholipid biosynthetic process [GO:0071072]; is a type of regulation of phosphatidylcholine biosynthetic process [GO:2001245]; negatively regulates phosphatidylcholine biosynthetic process [GO:0006656] Also known as: negative regulation of phosphatidylcholine anabolism, negative regulation of phosphatidylcholine biosynthesis, negative regulation of phosphatidylcholine formation, negative regulation of phosphatidylcholine synthesis